{
  "gene": "UniProtKB:Q6UXI9",
  "gene_name": "Nephronectin",
  "term_label": "Unknown biological process",
  "term_id": "UNKNOWN:0002",
  "gene_symbol": "NPNT"
}